{
  "gene_symbol": "PDE3B",
  "gene": "UniProtKB:Q13370",
  "gene_name": "cGMP-inhibited 3',5'-cyclic phosphodiesterase 3B",
  "term_id": "GO:0004115",
  "term_label": "3',5'-cyclic-AMP phosphodiesterase activity"
}